{
  "gene": "UniProtKB:Q96Q07",
  "term_id": "GO:0008344",
  "gene_symbol": "BTBD9",
  "term_label": "adult locomotory behavior",
  "gene_name": "BTB_POZ domain-containing protein 9"
}